{
  "gene_name": "Homeobox protein Hox-B7",
  "term_label": "DNA-binding transcription factor activity, RNA polymerase II-specific",
  "gene": "UniProtKB:P09629",
  "term_id": "GO:0000981",
  "gene_symbol": "HOXB7"
}